{
  "gene_name": "Vascular endothelial growth factor receptor 2",
  "term_label": "plasma membrane",
  "gene_symbol": "KDR",
  "term_id": "GO:0005886",
  "gene": "UniProtKB:P35968"
}